{
  "term_id": "GO:0030425",
  "gene": "UniProtKB:Q9UBB6",
  "term_label": "dendrite",
  "gene_symbol": "NCDN",
  "gene_name": "Neurochondrin"
}